{
  "gene_symbol": "TIMD4",
  "gene": "UniProtKB:Q96H15",
  "term_label": "phosphatidylserine binding",
  "term_id": "GO:0001786",
  "gene_name": "T-cell immunoglobulin and mucin domain-containing protein 4"
}